{
  "term_label": "urocanate hydratase activity",
  "gene_symbol": "UROC1",
  "gene_name": "Urocanate hydratase",
  "term_id": "GO:0016153",
  "gene": "UniProtKB:Q96N76"
}